{
  "gene_symbol": "NT5C3A",
  "term_label": "5'-nucleotidase activity",
  "term_id": "GO:0008253",
  "gene": "UniProtKB:Q9H0P0",
  "gene_name": "Cytosolic 5'-nucleotidase 3A"
}